{
  "gene_name": "Leukocyte immunoglobulin-like receptor subfamily B member 4",
  "gene_symbol": "LILRB4",
  "term_id": "GO:0032396",
  "gene": "UniProtKB:Q8NHJ6",
  "term_label": "inhibitory MHC class I receptor activity"
}